{
  "term_label": "cyclosporin A binding",
  "gene_name": "Peptidyl-prolyl cis-trans isomerase A-like 4E",
  "gene": "UniProtKB:A0A075B759",
  "term_id": "GO:0016018",
  "gene_symbol": "PPIAL4E"
}